regulation of spindle assembly [GO:0090169] (BP) Relationships: is a type of regulation of spindle organization [GO:0090224]; is a type of GO:1902115; regulates spindle assembly [GO:0051225] Sources: GOC:ascb_2009, GOC:dph, GOC:tb Also known as: regulation of spindle formation Definition: Any process that modulates the rate, frequency or extent of spindle assembly. Spindle assembly is the aggregation, arrangement and bonding together of a set of components to form the spindle, the array of microtubules and associated molecules that serves to move duplicated chromosomes apart. Subtypes: regulation of mitotic spindle assembly [GO:1901673], negative regulation of spindle assembly [GO:1905831], positive regulation of spindle assembly [GO:1905832]